anaerobic toluene catabolic process [GO:0046254] (biological process) Also known as: anaerobic toluene breakdown, anaerobic toluene catabolism, anaerobic toluene degradation Relationships: is a type of toluene catabolic process [GO:0042203] Definition: The chemical reactions and pathways resulting in the breakdown of toluene, a volatile monoaromatic hydrocarbon found in crude petroleum and petroleum products, in the absence of oxygen. Sources: GOC:ai